{
  "gene_symbol": "SRRD",
  "term_label": "Unknown molecular function",
  "term_id": "UNKNOWN:0001",
  "gene_name": "SRR1-like protein",
  "gene": "UniProtKB:Q9UH36"
}